{
  "gene_name": "Low affinity immunoglobulin gamma Fc region receptor II-c",
  "gene_symbol": "FCGR2C",
  "term_id": "GO:0009897",
  "term_label": "external side of plasma membrane",
  "gene": "UniProtKB:P31995"
}